{
  "term_id": "GO:0003729",
  "term_label": "mRNA binding",
  "gene_name": "Probable RNA-binding protein 19",
  "gene_symbol": "RBM19",
  "gene": "UniProtKB:Q9Y4C8"
}